{
  "gene_name": "Rho GTPase-activating protein 20",
  "gene": "UniProtKB:Q9P2F6",
  "term_id": "GO:0005096",
  "term_label": "GTPase activator activity",
  "gene_symbol": "ARHGAP20"
}